{
  "gene": "UniProtKB:P23743",
  "term_id": "GO:0006654",
  "term_label": "phosphatidic acid biosynthetic process",
  "gene_symbol": "DGKA",
  "gene_name": "Diacylglycerol kinase alpha"
}